HDL-containing protein-lipid-RNA complex [GO:1990685] (cellular component) Note: Examples of HDL-containing protein-lipid-RNA complexes are described in PMID:21423178 and PMID:23559634, both showing evidence that high-density lipoproteins (HDL) transport endogenous microRNAs (miRNAs) and deliver them to recipient cells with functional targeting capabilities. Also see fig. 1 in the review PMID:22028337. Not to be confused with GO:0034364 'high-density lipoprotein particle', which describes complexes of proteins and lipids only, without RNAs. Relationships: is a type of GO:1990684 Definition: A protein-lipid-RNA complex containing separate high-density lipoprotein (HDL), lipid and RNA molecules. Separate in this context means not covalently bound to each other. References: PMID:21423178, PMID:23559634 Sources: GOC:vesicles